{
  "gene_symbol": "EHMT1",
  "term_label": "epigenetic regulation of gene expression",
  "term_id": "GO:0040029",
  "gene_name": "Histone-lysine N-methyltransferase EHMT1",
  "gene": "UniProtKB:Q9H9B1"
}